{
  "gene_symbol": "ANKRD16",
  "term_label": "Unknown biological process",
  "gene": "UniProtKB:Q6P6B7",
  "term_id": "UNKNOWN:0002",
  "gene_name": "Ankyrin repeat domain-containing protein 16"
}